{
  "gene_symbol": "CXCR6",
  "gene": "UniProtKB:O00574",
  "term_id": "GO:0007204",
  "term_label": "positive regulation of cytosolic calcium ion concentration",
  "gene_name": "C-X-C chemokine receptor type 6"
}